{
  "term_id": "UNKNOWN:0003",
  "gene": "UniProtKB:Q96SI9",
  "term_label": "Unknown cellular component",
  "gene_symbol": "STRBP",
  "gene_name": "Spermatid perinuclear RNA-binding protein"
}